pyrimidine deoxyribonucleoside metabolic process [GO:0046125] (biological process) Definition: The chemical reactions and pathways involving any one of a family of organic molecules consisting of a pyrimidine base covalently bonded to a sugar deoxyribose (a deoxyribonucleoside). Relationships: is a type of pyrimidine nucleoside metabolic process [GO:0006213]; is a type of deoxyribonucleoside metabolic process [GO:0009120] Also known as: pyrimidine deoxyribonucleoside metabolism Sources: GOC:ai Subtypes: pyrimidine deoxyribonucleoside interconversion [GO:0019690], GO:0046092, deoxyuridine metabolic process [GO:0046096], thymidine metabolic process [GO:0046104], pyrimidine deoxyribonucleoside biosynthetic process [GO:0046126], pyrimidine deoxyribonucleoside catabolic process [GO:0046127]